{
  "gene_name": "E3 ubiquitin-protein ligase SH3RF1",
  "gene": "UniProtKB:Q7Z6J0",
  "term_id": "GO:0001764",
  "gene_symbol": "SH3RF1",
  "term_label": "neuron migration"
}